natural killer cell lectin-like receptor binding [GO:0046703] (molecular function) Definition: Binding to a lectin-like natural killer cell receptor. Also known as: NK cell lectin-like receptor binding, KLRC4 receptor binding, NKG2D receptor binding Sources: GOC:ai Relationships: is a type of signaling receptor binding [GO:0005102]